{
  "term_id": "GO:0033700",
  "gene_symbol": "APOE",
  "gene": "UniProtKB:P02649",
  "term_label": "phospholipid efflux",
  "gene_name": "Apolipoprotein E"
}